{
  "gene_name": "Pregnancy-specific beta-1-glycoprotein 5",
  "gene": "UniProtKB:Q15238",
  "gene_symbol": "PSG5",
  "term_id": "GO:0005886",
  "term_label": "plasma membrane"
}